{
  "term_label": "lipoprotein transport",
  "gene_symbol": "CD36",
  "term_id": "GO:0042953",
  "gene_name": "Platelet glycoprotein 4",
  "gene": "UniProtKB:P16671"
}